{
  "gene_name": "A disintegrin and metalloproteinase with thrombospondin motifs 8",
  "term_id": "GO:0031012",
  "gene_symbol": "ADAMTS8",
  "term_label": "extracellular matrix",
  "gene": "UniProtKB:Q9UP79"
}